{
  "gene": "UniProtKB:Q96PN7",
  "term_label": "transcription corepressor activity",
  "gene_symbol": "TRERF1",
  "term_id": "GO:0003714",
  "gene_name": "Transcriptional-regulating factor 1"
}